{
  "gene_symbol": "RAB6C",
  "term_label": "endomembrane system",
  "gene_name": "Ras-related protein Rab-6C",
  "gene": "UniProtKB:Q9H0N0",
  "term_id": "GO:0012505"
}